{
  "gene": "UniProtKB:P62258",
  "gene_symbol": "YWHAE",
  "term_label": "regulation of mitotic cell cycle",
  "gene_name": "14-3-3 protein epsilon",
  "term_id": "GO:0007346"
}